negative regulation of epithelial cell proliferation involved in prostate gland development [GO:0060770] (biological process) Definition: Any process that decreases the rate, frequency or extent of epithelial cell proliferation that contributes to the progression of the prostate gland over time. Relationships: is a type of negative regulation of epithelial cell proliferation [GO:0050680]; is a type of negative regulation of developmental process [GO:0051093]; is a type of GO:0051241; is a type of regulation of epithelial cell proliferation involved in prostate gland development [GO:0060768]; is a type of GO:2000242; negatively regulates epithelial cell proliferation involved in prostate gland development [GO:0060767] Sources: GOC:dph